{
  "gene": "UniProtKB:Q9Y5P4",
  "term_label": "ER to Golgi ceramide transport",
  "term_id": "GO:0035621",
  "gene_symbol": "CERT1",
  "gene_name": "Ceramide transfer protein"
}